response to flooding [GO:0009413] (biological process) Note: Note that this term should not be confused with 'response to deep water ; GO:0030912'. Flooding refers to short-term immersion, whereas 'response to deep water ; GO:0030912' refers to standing in water throughout an organism's life cycle. Sources: GOC:lr Relationships: is a type of response to stress [GO:0006950]; is_a response to water [GO:0009415] Definition: Any process that results in a change in state or activity of a cell or an organism (in terms of movement, secretion, enzyme production, gene expression, etc.) as a result of a stimulus indicating flooding, short-term immersion in water.